{
  "term_label": "plasma membrane",
  "gene_name": "Short transient receptor potential channel 3",
  "gene_symbol": "TRPC3",
  "term_id": "GO:0005886",
  "gene": "UniProtKB:Q13507"
}